positive regulation of regulatory T cell differentiation [GO:0045591] (biological process) Definition: Any process that activates or increases the frequency, rate or extent of differentiation of regulatory T cells. Relationships: is a type of positive regulation of T cell differentiation [GO:0045582]; is a type of regulation of regulatory T cell differentiation [GO:0045589]; positively regulates regulatory T cell differentiation [GO:0045066] Note: Note that immunologists typically use the word 'development' to refer to cells of B or T cell lineages undergoing the process that GO describes as 'cell differentiation'. Sources: ISBN:0781735149 Also known as: positive regulation of regulatory T lymphocyte differentiation, positive regulation of regulatory T-cell differentiation, positive regulation of regulatory T-lymphocyte differentiation, positive regulation of suppressor T cell differentiation, positive regulation of suppressor T-cell differentiation, up regulation of regulatory T cell differentiation, up-regulation of regulatory T cell differentiation, upregulation of regulatory T cell differentiation, activation of regulatory T cell differentiation, stimulation of regulatory T cell differentiation, positive regulation of regulatory T cell development Subtypes: GO:0032831